{
  "gene": "UniProtKB:Q9H257",
  "term_label": "signal transduction",
  "gene_symbol": "CARD9",
  "term_id": "GO:0007165",
  "gene_name": "Caspase recruitment domain-containing protein 9"
}